norepinephrine secretion [GO:0048243] (biological process) Regulation: negatively regulated by GO:0010700; positively regulated by positive regulation of norepinephrine secretion [GO:0010701]; regulated by regulation of norepinephrine secretion [GO:0014061] Subtypes: norepinephrine secretion, neurotransmission [GO:0061533] Sources: GOC:ef, GOC:jid Relationships: is a type of norepinephrine transport [GO:0015874]; is a type of signal release [GO:0023061]; is a type of GO:0050432 Definition: The regulated release of norepinephrine by a cell. Norepinephrine is a catecholamine and it acts as a hormone and as a neurotransmitter of most of the sympathetic nervous system. Also known as: noradrenaline secretion